{
  "term_label": "mechanosensitive monoatomic ion channel activity",
  "gene_name": "Transmembrane channel-like protein 3",
  "term_id": "GO:0008381",
  "gene": "UniProtKB:Q7Z5M5",
  "gene_symbol": "TMC3"
}